{
  "term_id": "UNKNOWN:0001",
  "gene": "UniProtKB:A2CJ06",
  "gene_symbol": "DYTN",
  "term_label": "Unknown molecular function",
  "gene_name": "Dystrotelin"
}